{
  "gene": "UniProtKB:Q5VZ46",
  "gene_symbol": "KIAA1614",
  "gene_name": "Uncharacterized protein KIAA1614",
  "term_label": "regulation of cellular localization",
  "term_id": "GO:0060341"
}